{
  "gene_symbol": "LCK",
  "term_id": "GO:0007169",
  "term_label": "cell surface receptor protein tyrosine kinase signaling pathway",
  "gene": "UniProtKB:P06239",
  "gene_name": "Tyrosine-protein kinase Lck"
}